{
  "gene_symbol": "SCFD2",
  "term_label": "vesicle-mediated transport",
  "gene": "UniProtKB:Q8WU76",
  "gene_name": "Sec1 family domain-containing protein 2",
  "term_id": "GO:0016192"
}